{
  "gene": "UniProtKB:Q9HB90",
  "gene_name": "Ras-related GTP-binding protein C",
  "gene_symbol": "RRAGC",
  "term_label": "Gtr1-Gtr2 GTPase complex",
  "term_id": "GO:1990131"
}